{
  "gene": "UniProtKB:Q9NZQ0",
  "gene_name": "DnaJ homolog subfamily C member 27",
  "gene_symbol": "DNAJC27",
  "term_label": "Unknown cellular component",
  "term_id": "UNKNOWN:0003"
}